{
  "gene_name": "Kallikrein-9",
  "gene_symbol": "KLK9",
  "gene": "UniProtKB:Q9UKQ9",
  "term_id": "GO:0004252",
  "term_label": "serine-type endopeptidase activity"
}